quinolinate metabolic process [GO:0046874] (biological process) Definition: The chemical reactions and pathways involving quinolinate, the anion of quinolinic acid, also known as 2,3-pyridinedicarboxylic acid. Sources: GOC:ai Also known as: quinolinate metabolism Relationships: is a type of dicarboxylic acid metabolic process [GO:0043648]; is a type of GO:0072524 Subtypes: quinolinate biosynthetic process [GO:0019805], quinolinate catabolic process [GO:0034213]